{
  "gene": "UniProtKB:Q86V97",
  "term_id": "GO:1990756",
  "gene_symbol": "KBTBD6",
  "gene_name": "Kelch repeat and BTB domain-containing protein 6",
  "term_label": "ubiquitin-like ligase-substrate adaptor activity"
}